{
  "gene_name": "Cadherin-22",
  "gene_symbol": "CDH22",
  "gene": "UniProtKB:Q9UJ99",
  "term_id": "GO:0000902",
  "term_label": "cell morphogenesis"
}